{
  "term_label": "maturation of SSU-rRNA",
  "gene_name": "Small ribosomal subunit protein eS28",
  "gene": "UniProtKB:P62857",
  "gene_symbol": "RPS28",
  "term_id": "GO:0030490"
}